{
  "term_label": "voltage-gated potassium channel activity",
  "term_id": "GO:0005249",
  "gene": "UniProtKB:Q9Y3Q4",
  "gene_name": "Potassium_sodium hyperpolarization-activated cyclic nucleotide-gated channel 4",
  "gene_symbol": "HCN4"
}